{
  "gene_name": "Transmembrane protein 203",
  "gene_symbol": "TMEM203",
  "term_label": "endoplasmic reticulum",
  "term_id": "GO:0005783",
  "gene": "UniProtKB:Q969S6"
}